{
  "term_id": "GO:0005262",
  "gene_name": "Transient receptor potential cation channel subfamily V member 4",
  "gene_symbol": "TRPV4",
  "gene": "UniProtKB:Q9HBA0",
  "term_label": "calcium channel activity"
}